{
  "term_label": "Unknown cellular component",
  "gene_symbol": "KRTAP23-1",
  "term_id": "UNKNOWN:0003",
  "gene_name": "Keratin-associated protein 23-1",
  "gene": "UniProtKB:A1A580"
}